{
  "gene_symbol": "CFAP298",
  "gene": "UniProtKB:P57076",
  "term_id": "UNKNOWN:0003",
  "gene_name": "Cilia- and flagella-associated protein 298",
  "term_label": "Unknown cellular component"
}